{
  "term_label": "U4/U6 x U5 tri-snRNP complex",
  "gene": "UniProtKB:O95777",
  "gene_name": "U6 snRNA-associated Sm-like protein LSm8",
  "gene_symbol": "LSM8",
  "term_id": "GO:0046540"
}